cellotriose binding [GO:0044583] (molecular function) Definition: Binding to cellotriose. Sources: GOC:mengo_curators, GOC:tt Relationships: is a type of trisaccharide binding [GO:0048031]